{
  "gene_symbol": "CHRM1",
  "gene_name": "Muscarinic acetylcholine receptor M1",
  "term_label": "G protein-coupled acetylcholine receptor activity",
  "term_id": "GO:0016907",
  "gene": "UniProtKB:P11229"
}